{
  "gene": "UniProtKB:Q13123",
  "gene_symbol": "IK",
  "term_label": "mRNA splicing, via spliceosome",
  "gene_name": "Protein Red",
  "term_id": "GO:0000398"
}